{
  "term_id": "GO:0005102",
  "gene": "UniProtKB:Q6UW32",
  "gene_name": "Insulin growth factor-like family member 1",
  "term_label": "signaling receptor binding",
  "gene_symbol": "IGFL1"
}